PEP carboxykinase C4 photosynthesis [GO:0009764] (biological process) Relationships: is a type of C4 photosynthesis [GO:0009760] Definition: The process of C4 photosynthesis, as it occurs in plants in which the enzyme decarboxylating C4 acids in the bundle sheath is phosphoenolpyruvate carboxykinase (PEPCK). References: PMID:11788762